{
  "gene": "UniProtKB:P17612",
  "gene_symbol": "PRKACA",
  "term_label": "nucleus",
  "term_id": "GO:0005634",
  "gene_name": "cAMP-dependent protein kinase catalytic subunit alpha"
}